{
  "gene_symbol": "FRZB",
  "term_label": "Wnt-protein binding",
  "term_id": "GO:0017147",
  "gene": "UniProtKB:Q92765",
  "gene_name": "Secreted frizzled-related protein 3"
}